3-chlorobenzoate-4,5-oxygenase activity [GO:0102044] (MF) Sources: GOC:pz Relationships: is a type of GO:0016708 Definition: Catalysis of the reaction: 3-chlorobenzoate + O2 + a reduced electron acceptor = 3-chlorobenzoate-cis-4,5-diol + an oxidized electron acceptor.